cerebellar mossy fiber [GO:0044300] (cellular component) Also known as: cerebellar mossy fibre Definition: An axon arising from cerebellar projecting cells in the cochlea, vestibular nuclei, spinal cord, reticular formation, cerebellar nuclei and basilar pontine nuclei. Mossy fibers enter through all three cerebellar peduncles and send collaterals to the deep cerebellar nuclei, then branch in the white matter and terminate in the granule cell layer. Through this branching, a given mossy fiber can innervate several folia. Mossy fibers synapse on granule cells. The synaptic contacts are made at enlargements along the length of the mossy fiber called mossy fiber rosettes. The enlargements of the rosettes give the axons a mossy-looking appearance in Golgi stained preparations. Relationships: is a type of axon [GO:0030424] Sources: NIF_Subcellular:nlx_subcell_20090209